prosthetic group biosynthetic process [GO:0051191] (BP) Sources: GOC:ai Definition: The chemical reactions and pathways resulting in the formation of a prosthetic group, the non-amino acid portion of certain protein molecules. Prosthetic groups may be inorganic or organic and are usually required for the biological activity of the protein. Also known as: coenzyme and prosthetic group biosynthesis, coenzyme and prosthetic group biosynthetic process, prosthetic group anabolism, prosthetic group biosynthesis, prosthetic group formation, prosthetic group synthesis Relationships: is a type of biosynthetic process [GO:0009058]; is a type of prosthetic group metabolic process [GO:0051189]; is part of macromolecule biosynthetic process [GO:0009059]